{
  "gene_name": "Short-chain dehydrogenase_reductase family 9C member 7",
  "term_label": "steroid metabolic process",
  "term_id": "GO:0008202",
  "gene": "UniProtKB:Q8NEX9",
  "gene_symbol": "SDR9C7"
}